{
  "gene_name": "Anterior gradient protein 2 homolog",
  "term_label": "Unknown biological process",
  "gene": "UniProtKB:O95994",
  "gene_symbol": "AGR2",
  "term_id": "UNKNOWN:0002"
}